{
  "gene_name": "Olfactory receptor 8U3",
  "gene_symbol": "OR8U3",
  "term_label": "Unknown biological process",
  "term_id": "UNKNOWN:0002",
  "gene": "UniProtKB:Q8NH85"
}